{
  "gene_name": "Protein Shroom3",
  "term_label": "adherens junction",
  "gene_symbol": "SHROOM3",
  "term_id": "GO:0005912",
  "gene": "UniProtKB:Q8TF72"
}